{
  "gene_symbol": "RNF7",
  "term_label": "protein ubiquitination",
  "term_id": "GO:0016567",
  "gene": "UniProtKB:Q9UBF6",
  "gene_name": "RING-box protein 2"
}